{
  "term_id": "GO:0000981",
  "term_label": "DNA-binding transcription factor activity, RNA polymerase II-specific",
  "gene": "UniProtKB:Q99607",
  "gene_symbol": "ELF4",
  "gene_name": "ETS-related transcription factor Elf-4"
}